{
  "gene_symbol": "HCN2",
  "gene_name": "Potassium_sodium hyperpolarization-activated cyclic nucleotide-gated channel 2",
  "term_id": "GO:0035725",
  "gene": "UniProtKB:Q9UL51",
  "term_label": "sodium ion transmembrane transport"
}